{
  "gene_symbol": "U2SURP",
  "gene": "UniProtKB:O15042",
  "gene_name": "U2 snRNP-associated SURP motif-containing protein",
  "term_id": "GO:0005634",
  "term_label": "nucleus"
}